{
  "gene_symbol": "KLHL22",
  "term_label": "proteasome-mediated ubiquitin-dependent protein catabolic process",
  "gene_name": "Kelch-like protein 22",
  "gene": "UniProtKB:Q53GT1",
  "term_id": "GO:0043161"
}